{
  "gene_name": "Soluble scavenger receptor cysteine-rich domain-containing protein SSC5D",
  "term_id": "GO:0005044",
  "gene": "UniProtKB:A1L4H1",
  "gene_symbol": "SSC5D",
  "term_label": "scavenger receptor activity"
}